{
  "gene_symbol": "CYFIP2",
  "term_id": "GO:0030031",
  "gene_name": "Cytoplasmic FMR1-interacting protein 2",
  "gene": "UniProtKB:Q96F07",
  "term_label": "cell projection assembly"
}